vacuolar membrane [GO:0005774] (cellular component) Subtypes: autophagosome membrane [GO:0000421], plant-type vacuole membrane [GO:0009705], contractile vacuolar membrane [GO:0031164], lytic vacuole membrane [GO:0098852] Definition: The lipid bilayer surrounding the vacuole and separating its contents from the cytoplasm of the cell. Sources: GOC:ai Relationships: is a type of GO:0098588; is part of GO:0005773